{
  "term_label": "protein phosphatase binding",
  "term_id": "GO:0019903",
  "gene_symbol": "MYO16",
  "gene_name": "Unconventional myosin-XVI",
  "gene": "UniProtKB:Q9Y6X6"
}